regulation of rRNA catabolic process [GO:1902374] (biological process) References: PMID:20160119 Sources: GOC:TermGenie, GOC:bf Also known as: regulation of rRNA breakdown, regulation of rRNA catabolism, regulation of rRNA degradation Subtypes: regulation of rRNA stability [GO:0044357] Relationships: is a type of regulation of catabolic process [GO:0009894]; is a type of GO:0051252; RO_0002211 rRNA catabolic process [GO:0016075] Definition: Any process that modulates the frequency, rate or extent of rRNA catabolic process.